{
  "gene_name": "Uncharacterized protein C1orf141",
  "term_label": "Unknown biological process",
  "term_id": "UNKNOWN:0002",
  "gene": "UniProtKB:Q5JVX7",
  "gene_symbol": "C1orf141"
}